neuron maturation [GO:0042551] (biological process) Regulation: regulated by GO:0014041; positively regulated by GO:0014042; negatively regulated by negative regulation of neuron maturation [GO:0014043] Definition: A developmental process, independent of morphogenetic (shape) change, that is required for a neuron to attain its fully functional state. Sources: GOC:dph, GOC:jl Subtypes: neuron remodeling [GO:0016322] Relationships: is_a cell maturation [GO:0048469]; is part of neuron development [GO:0048666]